{
  "gene_name": "Transcription factor SOX-2",
  "gene_symbol": "SOX2",
  "gene": "UniProtKB:P48431",
  "term_id": "GO:0005634",
  "term_label": "nucleus"
}